{
  "gene_name": "Glycoprotein hormones alpha chain",
  "gene": "UniProtKB:P01215",
  "term_label": "G protein-coupled receptor signaling pathway",
  "gene_symbol": "CGA",
  "term_id": "GO:0007186"
}